{
  "term_label": "microtubule cytoskeleton organization",
  "gene_symbol": "PPP2R3C",
  "term_id": "GO:0000226",
  "gene_name": "Serine_threonine-protein phosphatase 2A regulatory subunit B'' subunit gamma",
  "gene": "UniProtKB:Q969Q6"
}